{
  "gene": "UniProtKB:P13928",
  "gene_symbol": "ANXA8",
  "term_label": "sarcolemma",
  "term_id": "GO:0042383",
  "gene_name": "Annexin A8"
}